{
  "term_label": "Unknown cellular component",
  "gene_name": "Plasmalemma vesicle-associated protein",
  "gene": "UniProtKB:Q9BX97",
  "gene_symbol": "PLVAP",
  "term_id": "UNKNOWN:0003"
}